positive regulation of pyloric antrum smooth muscle contraction [GO:0120072] (biological process) Definition: Any process that increases the frequency, rate or extent of any pyloric antrum smooth muscle contraction. Relationships: is a type of regulation of pyloric antrum smooth muscle contraction [GO:0120071]; is a type of positive regulation of gastro-intestinal system smooth muscle contraction [GO:1904306]; positively regulates pyloric antrum smooth muscle contraction [GO:0120065] References: PMID:15890336 Sources: GOC:sl